{
  "term_label": "transmitter-gated monoatomic ion channel activity involved in regulation of postsynaptic membrane potential",
  "gene_name": "Glutamate receptor ionotropic, NMDA 2B",
  "term_id": "GO:1904315",
  "gene": "UniProtKB:Q13224",
  "gene_symbol": "GRIN2B"
}